{
  "term_id": "UNKNOWN:0002",
  "term_label": "Unknown biological process",
  "gene_name": "Small integral membrane protein 7",
  "gene": "UniProtKB:Q9BQ49",
  "gene_symbol": "SMIM7"
}